{
  "term_id": "GO:0006956",
  "gene_symbol": "C8B",
  "term_label": "complement activation",
  "gene_name": "Complement component C8 beta chain",
  "gene": "UniProtKB:P07358"
}